{
  "gene_symbol": "GRID1",
  "gene_name": "Glutamate receptor ionotropic, delta-1",
  "term_id": "GO:0005886",
  "gene": "UniProtKB:Q9ULK0",
  "term_label": "plasma membrane"
}